{
  "gene_name": "Aspartyl aminopeptidase",
  "gene": "UniProtKB:Q9ULA0",
  "gene_symbol": "DNPEP",
  "term_label": "Unknown molecular function",
  "term_id": "UNKNOWN:0001"
}